{
  "term_label": "Unknown cellular component",
  "gene_symbol": "MARCHF3",
  "term_id": "UNKNOWN:0003",
  "gene": "UniProtKB:Q86UD3",
  "gene_name": "E3 ubiquitin-protein ligase MARCHF3"
}